{
  "gene_symbol": "VIP",
  "gene": "UniProtKB:P01282",
  "gene_name": "VIP peptides",
  "term_id": "GO:0043005",
  "term_label": "neuron projection"
}